{
  "term_label": "plasma membrane",
  "term_id": "GO:0005886",
  "gene": "UniProtKB:Q9NP84",
  "gene_symbol": "TNFRSF12A",
  "gene_name": "Tumor necrosis factor receptor superfamily member 12A"
}